{
  "term_label": "Unknown cellular component",
  "term_id": "UNKNOWN:0003",
  "gene": "UniProtKB:Q96EG1",
  "gene_name": "Arylsulfatase G",
  "gene_symbol": "ARSG"
}